{
  "gene": "UniProtKB:Q3MHD2",
  "term_id": "UNKNOWN:0002",
  "gene_name": "Protein LSM12",
  "gene_symbol": "LSM12",
  "term_label": "Unknown biological process"
}